{
  "gene": "UniProtKB:Q8NHP8",
  "gene_name": "Putative phospholipase B-like 2",
  "term_label": "Unknown biological process",
  "term_id": "UNKNOWN:0002",
  "gene_symbol": "PLBD2"
}